{
  "gene_name": "Olfactory receptor 5L1",
  "gene_symbol": "OR5L1",
  "term_id": "GO:0004984",
  "gene": "UniProtKB:Q8NGL2",
  "term_label": "olfactory receptor activity"
}